{
  "gene": "UniProtKB:Q96EK7",
  "term_label": "nucleus",
  "gene_name": "Constitutive coactivator of peroxisome proliferator-activated receptor gamma",
  "gene_symbol": "FAM120B",
  "term_id": "GO:0005634"
}